{
  "gene": "UniProtKB:A0A494C1R9",
  "term_label": "chromatin",
  "gene_symbol": "TSPY9",
  "term_id": "GO:0000785",
  "gene_name": "Testis-specific Y-encoded protein 9"
}